{
  "gene_symbol": "SH2B1",
  "term_id": "GO:0035556",
  "term_label": "intracellular signal transduction",
  "gene": "UniProtKB:Q9NRF2",
  "gene_name": "SH2B adapter protein 1"
}